post-embryonic retina morphogenesis in camera-type eye [GO:0060060] (biological process) Sources: GOC:dgh, GOC:dph Definition: The process in which the anatomical structure of the retina is generated and organized in a camera-type eye during the post-embryonic life stage. Relationships: is a type of GO:0009886; is part of retina morphogenesis in camera-type eye [GO:0060042]